{
  "term_label": "nucleus",
  "gene_symbol": "ABRAXAS2",
  "gene": "UniProtKB:Q15018",
  "gene_name": "BRISC complex subunit Abraxas 2",
  "term_id": "GO:0005634"
}